{
  "gene": "UniProtKB:Q969U6",
  "gene_symbol": "FBXW5",
  "term_label": "Unknown molecular function",
  "term_id": "UNKNOWN:0001",
  "gene_name": "F-box_WD repeat-containing protein 5"
}